{
  "term_id": "GO:0005737",
  "gene_symbol": "CAPN1",
  "term_label": "cytoplasm",
  "gene_name": "Calpain-1 catalytic subunit",
  "gene": "UniProtKB:P07384"
}